{
  "term_id": "GO:1904262",
  "gene": "UniProtKB:P58004",
  "gene_symbol": "SESN2",
  "term_label": "negative regulation of TORC1 signaling",
  "gene_name": "Sestrin-2"
}